sulfuric ester hydrolase activity [GO:0008484] (molecular function) Subtypes: GO:0003943, arylsulfatase activity [GO:0004065], cerebroside-sulfatase activity [GO:0004098], iduronate-2-sulfatase activity [GO:0004423], GO:0004773, N-acetylglucosamine-6-sulfatase activity [GO:0008449], GO:0015024, linear primary-alkylsulfatase activity [GO:0018741], cellulose-polysulfatase activity [GO:0033886], chondro-4-sulfatase activity [GO:0033887], chondro-6-sulfatase activity [GO:0033888], N-sulfoglucosamine-3-sulfatase activity [GO:0033889], N-acetylgalactosamine-6-sulfatase activity [GO:0043890], choline-sulfatase activity [GO:0047753], D-lactate-2-sulfatase activity [GO:0047825], GO:0047871, glycosulfatase activity [GO:0047966], monomethyl-sulfatase activity [GO:0050106] Also known as: sulfatase activity, sulphuric ester hydrolase activity Relationships: is a type of hydrolase activity, acting on ester bonds [GO:0016788] Sources: GOC:ai Definition: Catalysis of the reaction: RSO-R' + H2O = RSOOH + R'H. This reaction is the hydrolysis of a sulfuric ester bond, an ester formed from sulfuric acid, O=SO(OH)2.